{
  "gene_name": "Putative chemokine-related protein FP248",
  "gene": "UniProtKB:Q71RG6",
  "term_label": "Unknown molecular function",
  "term_id": "UNKNOWN:0001",
  "gene_symbol": "FP248"
}